{
  "term_label": "ubiquitin protein ligase activity",
  "gene_name": "BRCA1-associated protein",
  "gene_symbol": "BRAP",
  "term_id": "GO:0061630",
  "gene": "UniProtKB:Q7Z569"
}